{
  "gene_symbol": "VIL1",
  "term_label": "actin polymerization or depolymerization",
  "gene": "UniProtKB:P09327",
  "gene_name": "Villin-1",
  "term_id": "GO:0008154"
}